{
  "gene_name": "t-SNARE domain-containing protein 1",
  "term_label": "endomembrane system",
  "gene": "UniProtKB:Q96NA8",
  "gene_symbol": "TSNARE1",
  "term_id": "GO:0012505"
}